negative regulation of leukocyte chemotaxis [GO:0002689] (BP) Sources: GOC:add Definition: Any process that stops, prevents, or reduces the frequency, rate, or extent of leukocyte chemotaxis. Also known as: down regulation of leukocyte chemotaxis, down-regulation of leukocyte chemotaxis, downregulation of leukocyte chemotaxis, negative regulation of immune cell chemotaxis, negative regulation of leucocyte chemotaxis, inhibition of leukocyte chemotaxis Subtypes: negative regulation of macrophage chemotaxis [GO:0010760], GO:0060755, negative regulation of granulocyte chemotaxis [GO:0071623], negative regulation of monocyte chemotaxis [GO:0090027], GO:1901624, negative regulation of dendritic cell chemotaxis [GO:2000509] Relationships: is a type of negative regulation of leukocyte migration [GO:0002686]; is_a regulation of leukocyte chemotaxis [GO:0002688]; is_a GO:0050922; negatively regulates leukocyte chemotaxis [GO:0030595]